{
  "gene": "UniProtKB:O14933",
  "gene_symbol": "UBE2L6",
  "gene_name": "Ubiquitin_ISG15-conjugating enzyme E2 L6",
  "term_label": "ubiquitin-dependent protein catabolic process",
  "term_id": "GO:0006511"
}